{
  "gene_name": "Protein c-Fos",
  "gene_symbol": "FOS",
  "gene": "UniProtKB:P01100",
  "term_id": "GO:0006357",
  "term_label": "regulation of transcription by RNA polymerase II"
}